{
  "gene_name": "Myeloblastin",
  "gene": "UniProtKB:P24158",
  "term_label": "neutrophil extravasation",
  "term_id": "GO:0072672",
  "gene_symbol": "PRTN3"
}